{
  "gene_name": "Multimerin-2",
  "term_id": "UNKNOWN:0001",
  "gene_symbol": "MMRN2",
  "gene": "UniProtKB:Q9H8L6",
  "term_label": "Unknown molecular function"
}